{
  "term_label": "protein folding",
  "term_id": "GO:0006457",
  "gene_name": "Prefoldin subunit 6",
  "gene": "UniProtKB:O15212",
  "gene_symbol": "PFDN6"
}